{
  "gene_name": "DH domain-containing protein",
  "term_label": "regulation of actin cytoskeleton organization",
  "gene_symbol": "LOC107987545",
  "term_id": "GO:0032956",
  "gene": "UniProtKB:A0A2R8YFR7"
}